{
  "gene": "UniProtKB:P49771",
  "term_id": "GO:0030971",
  "gene_name": "Fms-related tyrosine kinase 3 ligand",
  "gene_symbol": "FLT3LG",
  "term_label": "receptor tyrosine kinase binding"
}